positive regulation of sebum secreting cell proliferation [GO:1904004] (biological process) Relationships: is a type of positive regulation of epithelial cell proliferation [GO:0050679]; is a type of GO:1904002; positively regulates sebum secreting cell proliferation [GO:1990654] Definition: Any process that activates or increases the frequency, rate or extent of sebum secreting cell proliferation. Also known as: up regulation of sebum secreting cell proliferation, up-regulation of sebum secreting cell proliferation, upregulation of sebum secreting cell proliferation, activation of sebum secreting cell proliferation, activation of sebocyte proliferation, positive regulation of sebocyte proliferation, up regulation of sebocyte proliferation, up-regulation of sebocyte proliferation, upregulation of sebocyte proliferation References: PMID:16901790 Sources: GOC:TermGenie, GOC:hjd, GO_REF:0000058